{
  "gene": "UniProtKB:Q7Z4H9",
  "term_id": "GO:0005634",
  "gene_symbol": "FAM220A",
  "term_label": "nucleus",
  "gene_name": "Protein FAM220A"
}